{
  "term_label": "negative regulation of transcription by RNA polymerase II",
  "gene": "UniProtKB:Q9UIS9",
  "gene_name": "Methyl-CpG-binding domain protein 1",
  "term_id": "GO:0000122",
  "gene_symbol": "MBD1"
}